ketosteroid monooxygenase activity [GO:0047086] (molecular function) Relationships: is a type of oxidoreductase activity, acting on paired donors, with incorporation or reduction of molecular oxygen, NAD(P)H as one donor, and incorporation of one atom of oxygen [GO:0016709] Sources: EC:1.14.13.54, MetaCyc:1.14.13.54-RXN Definition: Catalysis of the reaction: O2 + NADPH + progesterone = H2O + NADP+ + testosterone acetate. Also known as: 17alpha-hydroxyprogesterone, NADPH2:oxygen oxidoreductase (20-hydroxylating, side-chain cleaving), androstenedione, NADPH2:oxygen oxidoreductase (17-hydroxylating, lactonizing), ketosteroid,NADPH:oxygen oxidoreductase (20-hydroxylating, ester-producing/20-hydroxylating, side-chain cleaving/17-hydroxylating, lactonizing), progesterone, NADPH2:oxygen oxidoreductase (20-hydroxylating, ester-producing), steroid-ketone monooxygenase activity